{
  "gene_symbol": "HOXB2",
  "gene_name": "Homeobox protein Hox-B2",
  "term_id": "GO:0000981",
  "gene": "UniProtKB:P14652",
  "term_label": "DNA-binding transcription factor activity, RNA polymerase II-specific"
}